{
  "gene_name": "PRAME family member 18",
  "gene_symbol": "PRAMEF18",
  "gene": "UniProtKB:Q5VWM3",
  "term_label": "proteasome-mediated ubiquitin-dependent protein catabolic process",
  "term_id": "GO:0043161"
}